{
  "gene": "UniProtKB:Q6MZZ7",
  "gene_name": "Calpain-13",
  "term_label": "cytoplasm",
  "gene_symbol": "CAPN13",
  "term_id": "GO:0005737"
}